{
  "gene_name": "Hydroperoxide isomerase ALOXE3",
  "gene_symbol": "ALOXE3",
  "gene": "UniProtKB:Q9BYJ1",
  "term_id": "GO:0019369",
  "term_label": "arachidonate metabolic process"
}